{
  "term_id": "GO:0006362",
  "gene_symbol": "POLR1F",
  "term_label": "transcription elongation by RNA polymerase I",
  "gene_name": "DNA-directed RNA polymerase I subunit RPA43",
  "gene": "UniProtKB:Q3B726"
}